{
  "term_label": "nucleus",
  "term_id": "GO:0005634",
  "gene_name": "Cbp_p300-interacting transactivator 2",
  "gene_symbol": "CITED2",
  "gene": "UniProtKB:Q99967"
}